{
  "term_id": "GO:0005484",
  "gene_name": "Synaptosomal-associated protein 23",
  "gene_symbol": "SNAP23",
  "term_label": "SNAP receptor activity",
  "gene": "UniProtKB:O00161"
}